{
  "gene_name": "H(+)_Cl(-) exchange transporter 5",
  "gene": "UniProtKB:P51795",
  "term_label": "plasma membrane",
  "term_id": "GO:0005886",
  "gene_symbol": "CLCN5"
}